{
  "gene": "UniProtKB:Q04206",
  "gene_symbol": "RELA",
  "term_label": "response to cytokine",
  "term_id": "GO:0034097",
  "gene_name": "Transcription factor p65"
}